{
  "gene_name": "Transformation_transcription domain-associated protein",
  "gene": "UniProtKB:Q9Y4A5",
  "term_label": "Unknown molecular function",
  "gene_symbol": "TRRAP",
  "term_id": "UNKNOWN:0001"
}